{
  "term_label": "Unknown cellular component",
  "gene": "UniProtKB:P0CE67",
  "term_id": "UNKNOWN:0003",
  "gene_symbol": "LINC02877",
  "gene_name": "Putative uncharacterized protein encoded by LINC02877"
}